{
  "term_label": "signal transduction",
  "gene": "UniProtKB:O43741",
  "gene_symbol": "PRKAB2",
  "gene_name": "5'-AMP-activated protein kinase subunit beta-2",
  "term_id": "GO:0007165"
}